tripeptidyl-peptidase activity [GO:0008240] (molecular function) Relationships: is a type of GO:0070008 Definition: Catalysis of the release of an N-terminal tripeptide from a polypeptide. Sources: GOC:mah